{
  "gene_symbol": "A0A8I5QKQ9",
  "term_label": "Unknown biological process",
  "gene_name": "Uncharacterized protein",
  "gene": "UniProtKB:A0A8I5QKQ9",
  "term_id": "UNKNOWN:0002"
}